{
  "term_label": "double-stranded RNA binding",
  "gene": "UniProtKB:Q8IY21",
  "gene_symbol": "DDX60",
  "term_id": "GO:0003725",
  "gene_name": "Probable ATP-dependent RNA helicase DDX60"
}